{
  "gene_symbol": "TMEM232",
  "term_label": "spermatid cytoplasm removal during spermiation of flagellated sperm",
  "gene": "UniProtKB:C9JQI7",
  "term_id": "GO:0160087",
  "gene_name": "Transmembrane protein 232"
}